protein kinase A catalytic subunit binding [GO:0034236] (molecular function) Relationships: is a type of protein kinase binding [GO:0019901]; is a type of GO:0051018 Sources: GOC:mah Also known as: PKA catalytic subunit binding Definition: Binding to one or both of the catalytic subunits of protein kinase A.